negative regulation of establishment or maintenance of cell polarity regulating cell shape [GO:2000770] (BP) Definition: Any process that stops, prevents or reduces the frequency, rate or extent of establishment or maintenance of cell polarity regulating cell shape. Relationships: is a type of negative regulation of cellular process [GO:0048523]; is a type of regulation of establishment or maintenance of cell polarity regulating cell shape [GO:2000769]; negatively regulates establishment or maintenance of cell polarity regulating cell shape [GO:0071963] Sources: GOC:mah Subtypes: negative regulation of establishment or maintenance of bipolar cell polarity regulating cell shape [GO:2000750], GO:2000783